{
  "gene": "UniProtKB:Q9C0C7",
  "term_id": "GO:0080008",
  "gene_name": "Activating molecule in BECN1-regulated autophagy protein 1",
  "term_label": "Cul4-RING E3 ubiquitin ligase complex",
  "gene_symbol": "AMBRA1"
}